{
  "gene_symbol": "TESC",
  "gene": "UniProtKB:Q96BS2",
  "gene_name": "Calcineurin B homologous protein 3",
  "term_label": "regulation of cell adhesion mediated by integrin",
  "term_id": "GO:0033628"
}